{
  "term_label": "actin filament organization",
  "gene_name": "Engulfment and cell motility protein 3",
  "gene": "UniProtKB:Q96BJ8",
  "gene_symbol": "ELMO3",
  "term_id": "GO:0007015"
}